{
  "gene_name": "Olfactory receptor 10G2",
  "gene": "UniProtKB:Q8NGC3",
  "term_label": "detection of chemical stimulus involved in sensory perception of smell",
  "gene_symbol": "OR10G2",
  "term_id": "GO:0050911"
}